{
  "gene_name": "Growth_differentiation factor 2",
  "term_id": "GO:0030509",
  "gene_symbol": "GDF2",
  "term_label": "BMP signaling pathway",
  "gene": "UniProtKB:Q9UK05"
}